{
  "term_id": "GO:0030488",
  "gene": "UniProtKB:Q13395",
  "term_label": "tRNA methylation",
  "gene_symbol": "TARBP1",
  "gene_name": "Probable methyltransferase TARBP1"
}